{
  "term_label": "small GTPase-mediated signal transduction",
  "term_id": "GO:0007264",
  "gene_name": "Rho guanine nucleotide exchange factor 2",
  "gene": "UniProtKB:Q92974",
  "gene_symbol": "ARHGEF2"
}